{
  "term_label": "regulation of transcription by RNA polymerase II",
  "gene": "UniProtKB:Q86SE9",
  "gene_name": "Polycomb group RING finger protein 5",
  "gene_symbol": "PCGF5",
  "term_id": "GO:0006357"
}